{
  "gene": "UniProtKB:Q13618",
  "gene_symbol": "CUL3",
  "term_label": "ubiquitin protein ligase binding",
  "term_id": "GO:0031625",
  "gene_name": "Cullin-3"
}